{
  "term_label": "cytosol",
  "gene": "UniProtKB:Q9C037",
  "term_id": "GO:0005829",
  "gene_name": "E3 ubiquitin-protein ligase TRIM4",
  "gene_symbol": "TRIM4"
}